{
  "gene_name": "Polypeptide N-acetylgalactosaminyltransferase 6",
  "gene": "UniProtKB:Q8NCL4",
  "term_label": "polypeptide N-acetylgalactosaminyltransferase activity",
  "term_id": "GO:0004653",
  "gene_symbol": "GALNT6"
}